{
  "gene_symbol": "ZNF572",
  "gene": "UniProtKB:Q7Z3I7",
  "gene_name": "Zinc finger protein 572",
  "term_id": "GO:0002682",
  "term_label": "regulation of immune system process"
}